{
  "gene_symbol": "NUP85",
  "gene": "UniProtKB:Q9BW27",
  "term_id": "GO:0031080",
  "gene_name": "Nuclear pore complex protein Nup85",
  "term_label": "nuclear pore outer ring"
}